{
  "term_label": "Unknown molecular function",
  "gene_name": "Dolichyl-diphosphooligosaccharide--protein glycosyltransferase subunit 1",
  "gene": "UniProtKB:P04843",
  "gene_symbol": "RPN1",
  "term_id": "UNKNOWN:0001"
}